{
  "term_label": "dynein intermediate chain binding",
  "gene": "UniProtKB:P63167",
  "gene_symbol": "DYNLL1",
  "term_id": "GO:0045505",
  "gene_name": "Dynein light chain 1, cytoplasmic"
}